regulation of diorcinol biosynthetic process [GO:1900655] (biological process) Sources: GOC:TermGenie, GOC:di Also known as: regulation of diorcinol anabolism, regulation of diorcinol biosynthesis, regulation of diorcinol formation, regulation of diorcinol synthesis Relationships: is a type of regulation of secondary metabolite biosynthetic process [GO:1900376]; regulates diorcinol biosynthetic process [GO:1900572] Definition: Any process that modulates the frequency, rate or extent of diorcinol biosynthetic process. Subtypes: negative regulation of diorcinol biosynthetic process [GO:1900656], GO:1900657